dehydroaustinol catabolic process [GO:1900562] (biological process) Sources: GOC:TermGenie, GOC:di Definition: The chemical reactions and pathways resulting in the breakdown of dehydroaustinol. Also known as: dehydroaustinol breakdown, dehydroaustinol catabolism, dehydroaustinol degradation Relationships: is a type of secondary metabolite catabolic process [GO:0090487]